bacterial nucleoid [GO:0043590] (cellular component) Sources: GOC:jl Relationships: is a type of nucleoid [GO:0009295]; is a type of intracellular membraneless organelle [GO:0043232] Definition: The region of a bacterial cell to which the DNA is confined.